{
  "term_label": "extracellular matrix",
  "gene_name": "Procollagen-lysine,2-oxoglutarate 5-dioxygenase 1",
  "gene_symbol": "PLOD1",
  "gene": "UniProtKB:Q02809",
  "term_id": "GO:0031012"
}